{
  "gene_symbol": "GEN1",
  "term_label": "Unknown cellular component",
  "gene_name": "Flap endonuclease GEN homolog 1",
  "gene": "UniProtKB:Q17RS7",
  "term_id": "UNKNOWN:0003"
}